{
  "gene_symbol": "HSPB2",
  "term_label": "response to heat",
  "term_id": "GO:0009408",
  "gene": "UniProtKB:Q16082",
  "gene_name": "Heat shock protein beta-2"
}